{
  "gene_symbol": "PRDX5",
  "gene": "UniProtKB:P30044",
  "term_id": "GO:0005777",
  "term_label": "peroxisome",
  "gene_name": "Peroxiredoxin-5, mitochondrial"
}